{
  "gene": "UniProtKB:O43482",
  "term_id": "GO:0005634",
  "term_label": "nucleus",
  "gene_symbol": "OIP5",
  "gene_name": "Protein Mis18-beta"
}